{
  "term_id": "GO:0015813",
  "gene": "UniProtKB:O75746",
  "gene_symbol": "SLC25A12",
  "term_label": "L-glutamate transmembrane transport",
  "gene_name": "Electrogenic aspartate_glutamate antiporter SLC25A12, mitochondrial"
}